{
  "gene_symbol": "SCP2D1",
  "gene_name": "SCP2 sterol-binding domain-containing protein 1",
  "term_label": "Unknown biological process",
  "term_id": "UNKNOWN:0002",
  "gene": "UniProtKB:Q9UJQ7"
}